{
  "gene_name": "Zinc finger protein GLI1",
  "term_id": "GO:0000981",
  "gene": "UniProtKB:P08151",
  "term_label": "DNA-binding transcription factor activity, RNA polymerase II-specific",
  "gene_symbol": "GLI1"
}